{
  "gene": "UniProtKB:Q9HC21",
  "term_label": "mitochondrial inner membrane",
  "gene_symbol": "SLC25A19",
  "gene_name": "Mitochondrial thiamine pyrophosphate carrier",
  "term_id": "GO:0005743"
}